haltere development [GO:0007482] (biological process) Definition: The process whose specific outcome is the progression of the haltere over time, from its formation to the mature structure. The haltere is the club-shaped 'balancers' found on each side of the metathorax among the true flies (Diptera). They are the much-modified hind wings. References: PMID:32659004 Sources: GOC:jid Relationships: is a type of GO:0048737; is part of haltere disc development [GO:0035216]